{
  "gene_name": "Protein maelstrom homolog",
  "term_label": "P granule",
  "gene": "UniProtKB:Q96JY0",
  "term_id": "GO:0043186",
  "gene_symbol": "MAEL"
}